positive regulation of platelet aggregation [GO:1901731] (BP) Definition: Any process that activates or increases the frequency, rate or extent of platelet aggregation. Platelet aggregation is the adhesion of one platelet to one or more other platelets via adhesion molecules. Sources: GOC:TermGenie, GOC:fj Relationships: is a type of positive regulation of homotypic cell-cell adhesion [GO:0034112]; is a type of regulation of platelet aggregation [GO:0090330]; positively regulates GO:0070527 Also known as: positive regulation of blood platelet aggregation, up regulation of blood platelet aggregation, up regulation of platelet aggregation, up-regulation of blood platelet aggregation, up-regulation of platelet aggregation, upregulation of blood platelet aggregation, upregulation of platelet aggregation, activation of blood platelet aggregation, activation of platelet aggregation, activation of thrombocyte aggregation, positive regulation of thrombocyte aggregation, up regulation of thrombocyte aggregation, up-regulation of thrombocyte aggregation, upregulation of thrombocyte aggregation